{
  "term_label": "Unknown cellular component",
  "gene_symbol": "ZBTB24",
  "term_id": "UNKNOWN:0003",
  "gene_name": "Zinc finger and BTB domain-containing protein 24",
  "gene": "UniProtKB:O43167"
}